{
  "gene_symbol": "GTF2H2",
  "term_label": "transcription factor TFIIH holo complex",
  "gene_name": "General transcription factor IIH subunit 2",
  "gene": "UniProtKB:Q13888",
  "term_id": "GO:0005675"
}